{
  "gene": "UniProtKB:O95178",
  "gene_name": "NADH dehydrogenase [ubiquinone] 1 beta subcomplex subunit 2, mitochondrial",
  "gene_symbol": "NDUFB2",
  "term_label": "Unknown molecular function",
  "term_id": "UNKNOWN:0001"
}